{
  "gene": "UniProtKB:P31260",
  "gene_name": "Homeobox protein Hox-A10",
  "gene_symbol": "HOXA10",
  "term_label": "nucleus",
  "term_id": "GO:0005634"
}